emboliform nucleus development [GO:0021737] (BP) Sources: GOC:cls, GOC:curators, GOC:dgh, GOC:dph, GOC:jid Definition: The process whose specific outcome is the progression of the emboliform nucleus over time, from its formation to the mature structure. Relationships: is a type of neural nucleus development [GO:0048857]; is part of cerebellum development [GO:0021549]